{
  "term_id": "GO:0005634",
  "term_label": "nucleus",
  "gene_name": "MOB kinase activator 2",
  "gene": "UniProtKB:Q70IA6",
  "gene_symbol": "MOB2"
}